{
  "gene_name": "Transcription factor HES-5",
  "term_id": "GO:0007219",
  "term_label": "Notch signaling pathway",
  "gene_symbol": "HES5",
  "gene": "UniProtKB:Q5TA89"
}